{
  "gene_symbol": "FBH1",
  "gene": "UniProtKB:Q8NFZ0",
  "gene_name": "F-box DNA helicase 1",
  "term_label": "double-strand break repair via homologous recombination",
  "term_id": "GO:0000724"
}